{
  "gene_name": "Putative adrenomedullin-5-like protein",
  "gene": "UniProtKB:C9JUS6",
  "term_id": "GO:0007189",
  "term_label": "adenylate cyclase-activating G protein-coupled receptor signaling pathway",
  "gene_symbol": "ADM5"
}